protein localization to medial cortical node [GO:1902577] (biological process) References: PMID:24127216 Sources: GOC:TermGenie Definition: A process in which a protein is transported to, or maintained in, a location within a medial cortical node. Relationships: is a type of protein localization to medial cortex [GO:0071574] Regulation: RO_0002211 by regulation of protein localization to medial cortical node [GO:0120046]; positively regulated by positive regulation of protein localization to medial cortical node [GO:0120047] Also known as: protein localisation in medial cortical node, protein localisation to medial cortical node, protein localization in medial cortical node